UDP-N-acetylglucosamine diphosphorylase activity [GO:0003977] (molecular function) Relationships: is a type of uridylyltransferase activity [GO:0070569] Definition: Catalysis of the reaction: N-acetyl-alpha-D-glucosamine 1-phosphate + UTP = diphosphate + UDP-N-acetyl-alpha-D-glucosamine. Sources: EC:2.7.7.23, RHEA:13509 Also known as: acetylglucosamine 1-phosphate uridylyltransferase, UDP-N-acetylglucosamine pyrophosphorylase activity, GlmU uridylyltransferase activity, N-acetylglucosamine-1-phosphate uridyltransferase activity, UDP-GlcNAc pyrophosphorylase activity, UDP-acetylglucosamine pyrophosphorylase activity, UTP:2-acetamido-2-deoxy-alpha-D-glucose-1-phosphate uridylyltransferase activity, UTP:N-acetyl-alpha-D-glucosamine-1-phosphate uridylyltransferase activity, uridine diphosphate-N-acetylglucosamine pyrophosphorylase activity, uridine diphosphoacetylglucosamine phosphorylase activity, uridine diphosphoacetylglucosamine pyrophosphorylase activity